{
  "term_id": "UNKNOWN:0001",
  "term_label": "Unknown molecular function",
  "gene_symbol": "A0A096LPG2",
  "gene_name": "Uncharacterized protein",
  "gene": "UniProtKB:A0A096LPG2"
}